{
  "gene_name": "Zinc finger CCHC domain-containing protein 13",
  "term_label": "single-stranded RNA binding",
  "term_id": "GO:0003727",
  "gene_symbol": "ZCCHC13",
  "gene": "UniProtKB:Q8WW36"
}